{
  "gene": "UniProtKB:A6NDU8",
  "term_label": "Unknown cellular component",
  "gene_symbol": "RIMOC1",
  "term_id": "UNKNOWN:0003",
  "gene_name": "RAB7A-interacting MON1-CCZ1 complex subunit 1"
}